{
  "term_label": "protein localization to plasma membrane",
  "gene_name": "Phosphofurin acidic cluster sorting protein 2",
  "gene_symbol": "PACS2",
  "gene": "UniProtKB:Q86VP3",
  "term_id": "GO:0072659"
}